{
  "gene_name": "Coiled-coil domain-containing protein 187",
  "gene_symbol": "CCDC187",
  "gene": "UniProtKB:A0A096LP49",
  "term_id": "UNKNOWN:0003",
  "term_label": "Unknown cellular component"
}